{
  "term_id": "UNKNOWN:0003",
  "term_label": "Unknown cellular component",
  "gene": "UniProtKB:Q8N2B8",
  "gene_symbol": "Q8N2B8",
  "gene_name": "Putative uncharacterized protein FLJ33534"
}